{
  "gene_symbol": "DPP10",
  "gene_name": "Inactive dipeptidyl peptidase 10",
  "term_id": "GO:0015459",
  "term_label": "potassium channel regulator activity",
  "gene": "UniProtKB:Q8N608"
}